{
  "term_id": "UNKNOWN:0001",
  "term_label": "Unknown molecular function",
  "gene_name": "Leucine-rich repeat, immunoglobulin-like domain and transmembrane domain-containing protein 2",
  "gene_symbol": "LRIT2",
  "gene": "UniProtKB:A6NDA9"
}